low-density lipoprotein particle remodeling [GO:0034374] (biological process) Definition: The acquisition, loss or modification of a protein or lipid within a low-density lipoprotein particle, including the hydrolysis of triglyceride by hepatic lipase, with the subsequent loss of free fatty acid, and the transfer of cholesterol esters from LDL to a triglyceride-rich lipoprotein particle by cholesteryl ester transfer protein (CETP), with the simultaneous transfer of triglyceride to LDL. Also known as: LDL remodeling, LDL remodelling, low-density lipoprotein particle remodelling, small dense LDL formation, small dense low-density lipoprotein particle formation Relationships: is a type of GO:0034369 Sources: GOC:BHF, GOC:expert_pt, GOC:mah, GOC:rl